{
  "term_id": "GO:0005525",
  "gene_name": "Cell division control protein 42 homolog",
  "term_label": "GTP binding",
  "gene_symbol": "CDC42",
  "gene": "UniProtKB:P60953"
}